{
  "gene": "UniProtKB:Q9Y4D1",
  "term_id": "UNKNOWN:0002",
  "gene_name": "Disheveled-associated activator of morphogenesis 1",
  "gene_symbol": "DAAM1",
  "term_label": "Unknown biological process"
}